{
  "term_id": "GO:0032475",
  "gene_name": "Proton channel OTOP1",
  "gene_symbol": "OTOP1",
  "gene": "UniProtKB:Q7RTM1",
  "term_label": "otolith formation"
}